{
  "gene": "UniProtKB:Q12837",
  "term_id": "UNKNOWN:0003",
  "gene_symbol": "POU4F2",
  "gene_name": "POU domain, class 4, transcription factor 2",
  "term_label": "Unknown cellular component"
}